L-alanine conjugated cholate hydrolase activity [GO:7770005] (molecular function) References: PMID:38326609 Sources: RHEA:79131 Definition: Catalysis of the reaction: cholate + L-alanine = L-alanocholate + H2O. Relationships: is a type of GO:7770003